{
  "gene_symbol": "PRRC2A",
  "gene": "UniProtKB:P48634",
  "term_id": "UNKNOWN:0003",
  "term_label": "Unknown cellular component",
  "gene_name": "Protein PRRC2A"
}